protein catabolic process at presynapse [GO:0140247] (biological process) Relationships: is a type of protein catabolic process at synapse [GO:0140246]; occurs in presynapse [GO:0098793] Definition: The chemical reactions and pathways resulting in the breakdown of a protein at a presynapse. References: PMID:27764673 Note: Note that this term was created for the SynGO project, and will be obsoleted when the SynGO annotations are made in Noctua.